{
  "term_id": "GO:0046512",
  "term_label": "sphingosine biosynthetic process",
  "gene_name": "Alkaline ceramidase 2",
  "gene_symbol": "ACER2",
  "gene": "UniProtKB:Q5QJU3"
}